{
  "term_id": "GO:0005849",
  "gene": "UniProtKB:O43809",
  "term_label": "mRNA cleavage factor complex",
  "gene_symbol": "NUDT21",
  "gene_name": "Cleavage and polyadenylation specificity factor subunit 5"
}